{
  "term_label": "Unknown cellular component",
  "gene": "UniProtKB:Q8N9H9",
  "gene_symbol": "C1orf127",
  "gene_name": "Uncharacterized protein C1orf127",
  "term_id": "UNKNOWN:0003"
}